actin filament severing activity [GO:0003789] (MF) Relationships: is a type of GO:0140776; is part of actin cytoskeleton organization [GO:0030036]; has part actin filament binding [GO:0051015] Also known as: actin depolymerizing activity References: PMID:11812157, PMID:23395798, PMID:23727096 Definition: Binding to an actin subunit and promoting its dissociation from an actin filament by a local change in actin subunit conformation and orientation, and severing of filaments.